horsetail-astral microtubule array [GO:0032117] (cellular component) Relationships: is a type of aster [GO:0005818]; is part of cortical microtubule cytoskeleton [GO:0030981] Definition: An array of astral microtubules that emanates from the spindle pole body during meiosis and facilitates horsetail nuclear movement. References: PMID:16111942 Sources: GOC:mah Also known as: HAA